{
  "gene_symbol": "PPM1A",
  "term_label": "protein serine/threonine phosphatase activity",
  "gene": "UniProtKB:P35813",
  "gene_name": "Protein phosphatase 1A",
  "term_id": "GO:0004722"
}